{
  "gene": "UniProtKB:Q9NRI5",
  "term_id": "GO:0007420",
  "gene_name": "Disrupted in schizophrenia 1 protein",
  "gene_symbol": "DISC1",
  "term_label": "brain development"
}